{
  "gene_symbol": "SDHD",
  "gene_name": "Succinate dehydrogenase [ubiquinone] cytochrome b small subunit, mitochondrial",
  "term_id": "GO:0006099",
  "term_label": "tricarboxylic acid cycle",
  "gene": "UniProtKB:O14521"
}